positive regulation of metanephric mesenchymal cell migration by platelet-derived growth factor receptor-beta signaling pathway [GO:0035793] (biological process) Also known as: positive regulation of metanephric mesenchymal cell migration by PDGF receptor-beta signaling pathway, positive regulation of metanephric mesenchymal cell migration by PDGFR-beta signaling pathway, positive regulation of metanephric mesenchymal cell migration by betaPDGF receptor signaling pathway, positive regulation of metanephric mesenchymal cell migration by platelet-derived growth factor receptor-beta signalling pathway Relationships: is a type of regulation of metanephric mesenchymal cell migration by platelet-derived growth factor receptor-beta signaling pathway [GO:1900238]; is a type of positive regulation of metanephric mesenchymal cell migration [GO:2000591] References: PMID:10734101 Sources: GOC:bf, GOC:mtg_kidney_jan10, GOC:yaf Definition: Any process that increases the frequency, rate or extent of metanephric mesenchymal cell migration resulting from the platelet-derived growth factor receptor-beta signaling pathway.